C2H2 zinc finger domain binding [GO:0070742] (molecular function) Definition: Binding to a C2H2-type zinc finger domain of a protein. The C2H2 zinc finger is the classical zinc finger domain, in which two conserved cysteines and histidines co-ordinate a zinc ion. Relationships: is a type of protein domain specific binding [GO:0019904] Sources: GOC:BHF, GOC:mah, Pfam:PF00096